ductus arteriosus closure [GO:0097070] (biological process) Regulation: regulated by regulation of ductus arteriosus closure [GO:1904335]; negatively regulated by GO:1904336; positively regulated by GO:1904337 Relationships: is a type of artery morphogenesis [GO:0048844] Sources: GOC:hw Definition: The morphogenesis process in which the ductus arteriosus changes to no longer permit blood flow after birth. The ductus arteriosus is the shunt between the aorta and the pulmonary artery which allows blood to bypass the fetus' lungs.